siRNA-mediated pericentric heterochromatin formation [GO:0140727] (biological process) Definition: The formation of pericentric heterochromatin by a process mediated by a small interfering RNA (siRNA). References: PMID:15289661 Also known as: RNAi-mediated heterochromatin assembly at centromere, siRNA dependent pericentric heterochromatin assembly, siRNA-dependent pericentric heterochromatin assembly, siRNA-dependent pericentric heterochromatin formation Relationships: is_a pericentric heterochromatin formation [GO:0031508]; is a type of siRNA-mediated heterochromatin formation [GO:0141194]